{
  "term_label": "regulation of G1/S transition of mitotic cell cycle",
  "gene": "UniProtKB:P61289",
  "gene_name": "Proteasome activator complex subunit 3",
  "gene_symbol": "PSME3",
  "term_id": "GO:2000045"
}